{
  "term_id": "UNKNOWN:0002",
  "gene_name": "Lysine-specific demethylase 9",
  "gene": "UniProtKB:Q5VWQ0",
  "gene_symbol": "RSBN1",
  "term_label": "Unknown biological process"
}